{
  "gene_name": "Interferon alpha-17",
  "term_label": "B cell activation involved in immune response",
  "gene_symbol": "IFNA17",
  "term_id": "GO:0002312",
  "gene": "UniProtKB:P01571"
}